palmitoyl-[glycerolipid] 7-desaturase activity [GO:0102843] (molecular function) Relationships: is a type of GO:0016717 Definition: Catalysis of the reaction: a 1-acyl-2-hexadecanoyl-glycerolipid + 2 H+ + O2 + 2 reduced [2Fe-2S]-[ferredoxin] = a 1-acyl-2-[(7Z)-hexadecenoyl]-glycerolipid + 2 H2O + 2 oxidized [2Fe-2S]-[ferredoxin]. Also known as: 1-18:2-2-16:0-monogalactosyldiacylglycerol desaturase activity (SN2-16:1 forming) Sources: RHEA:46756